{
  "term_label": "RNA polymerase II cis-regulatory region sequence-specific DNA binding",
  "gene_symbol": "HOXD4",
  "gene": "UniProtKB:P09016",
  "term_id": "GO:0000978",
  "gene_name": "Homeobox protein Hox-D4"
}